{
  "gene_name": "Putative gametogenetin-binding protein 1",
  "term_label": "Unknown cellular component",
  "gene_symbol": "GGNBP1",
  "gene": "UniProtKB:Q5YKI7",
  "term_id": "UNKNOWN:0003"
}